positive regulation of heart rate by neuronal norepinephrine [GO:0003113] (biological process) Relationships: is a type of positive regulation of heart rate by norepinephrine [GO:0003066] Also known as: positive regulation of heart rate by neuronal noradrenaline Definition: The process in which the secretion of norepinephrine released from nerve endings increases the rate of heart muscle contraction. Sources: GOC:mtg_cardio